histone glutaryltransferase activity [GO:0106229] (molecular function) Relationships: is a type of GO:0106228; is a type of histone modifying activity [GO:0140993] Definition: Catalysis of the reaction: glutaryl-CoA + histone = CoA + H+ + N6-glutaryl-histone. References: PMID:31542297 Sources: GOC:sp